{
  "term_label": "Unknown molecular function",
  "gene_symbol": "LEXM",
  "term_id": "UNKNOWN:0001",
  "gene_name": "Lymphocyte expansion molecule",
  "gene": "UniProtKB:Q3ZCV2"
}